{
  "gene_symbol": "AGBL5",
  "term_label": "metallocarboxypeptidase activity",
  "gene": "UniProtKB:Q8NDL9",
  "term_id": "GO:0004181",
  "gene_name": "Cytosolic carboxypeptidase-like protein 5"
}